{
  "gene_symbol": "LINC00310",
  "term_id": "UNKNOWN:0001",
  "gene_name": "Putative uncharacterized protein encoded by LINC00310",
  "term_label": "Unknown molecular function",
  "gene": "UniProtKB:P59036"
}